{
  "gene": "UniProtKB:Q96MM3",
  "gene_symbol": "ZFP42",
  "gene_name": "Zinc finger protein 42 homolog",
  "term_id": "GO:0000981",
  "term_label": "DNA-binding transcription factor activity, RNA polymerase II-specific"
}